inositol-3,5-bisdiphosphate-2,3,4,6-tetrakisphosphate 5-diphosphatase activity [GO:0052848] (molecular function) Relationships: is a type of inositol bisdiphosphate tetrakisphosphate diphosphatase activity [GO:0052841] References: PMID:10827188, PMID:11502751 Sources: RHEA:56312 Definition: Catalysis of the reaction: 3,5-bisdiphospho-1D-myo-inositol 2,3,4,6-tetrakisphosphate + H2O = 3-diphospho-1D-myo-inositol 1,2,4,5,6-pentakisphosphate + phosphate + 2 H+.